{
  "gene_name": "Alanine--tRNA ligase, mitochondrial",
  "term_label": "alanine-tRNA ligase activity",
  "term_id": "GO:0004813",
  "gene_symbol": "AARS2",
  "gene": "UniProtKB:Q5JTZ9"
}